{
  "term_id": "GO:0031105",
  "term_label": "septin complex",
  "gene": "UniProtKB:Q92599",
  "gene_symbol": "SEPTIN8",
  "gene_name": "Septin-8"
}